{
  "gene_symbol": "PTPRE",
  "gene": "UniProtKB:P23469",
  "term_id": "UNKNOWN:0003",
  "gene_name": "Receptor-type tyrosine-protein phosphatase epsilon",
  "term_label": "Unknown cellular component"
}